DNA ligase (NAD+) activity [GO:0003911] (molecular function) Relationships: is a type of GO:0003909 Also known as: DNA joinase activity, deoxyribonucleate ligase, deoxyribonucleic acid joinase, deoxyribonucleic acid ligase, deoxyribonucleic joinase, deoxyribonucleic ligase, polynucleotide ligase, DNA ligase (NAD), DNA repair enzyme activity, DNA-joining enzyme, deoxyribonucleic repair enzyme, deoxyribonucleic-joining enzyme, poly(deoxyribonucleotide):poly(deoxyribonucleotide) ligase (AMP-forming, NMN-forming), polydeoxyribonucleotide synthase (NAD(+)) activity, polydeoxyribonucleotide synthase (NAD), polydeoxyribonucleotide synthase (NAD+) activity, polynucleotide ligase (NAD(+)) activity, polynucleotide ligase (NAD), polynucleotide ligase (NAD+) activity, polynucleotide ligase (nicotinamide adenine dinucleotide), polynucleotide synthetase (nicotinamide adenine dinucleotide), polynucleotide synthetase activity Sources: EC:6.5.1.2 Definition: Catalysis of the reaction: NAD+ + deoxyribonucleotide(n) + deoxyribonucleotide(m) = AMP + nicotinamide nucleotide + deoxyribonucleotide(n+m).